{
  "gene": "UniProtKB:Q16650",
  "gene_symbol": "TBR1",
  "term_label": "RNA polymerase II cis-regulatory region sequence-specific DNA binding",
  "gene_name": "T-box brain protein 1",
  "term_id": "GO:0000978"
}